{
  "gene_name": "Myosin-3",
  "term_label": "actin filament binding",
  "term_id": "GO:0051015",
  "gene": "UniProtKB:P11055",
  "gene_symbol": "MYH3"
}